{
  "gene_name": "AF4_FMR2 family member 1",
  "gene": "UniProtKB:P51825",
  "term_id": "GO:0006355",
  "term_label": "regulation of DNA-templated transcription",
  "gene_symbol": "AFF1"
}